{
  "term_label": "Unknown cellular component",
  "gene_name": "Zinc finger SWIM domain-containing protein 3",
  "gene_symbol": "ZSWIM3",
  "term_id": "UNKNOWN:0003",
  "gene": "UniProtKB:Q96MP5"
}